{
  "term_label": "cytoplasm",
  "gene_symbol": "GCH1",
  "term_id": "GO:0005737",
  "gene": "UniProtKB:P30793",
  "gene_name": "GTP cyclohydrolase 1"
}